{
  "gene_name": "Intraflagellar transport protein 20 homolog",
  "gene": "UniProtKB:Q8IY31",
  "term_id": "GO:0005813",
  "term_label": "centrosome",
  "gene_symbol": "IFT20"
}